galanin-activated signaling pathway [GO:0090663] (biological process) Relationships: is a type of GO:0007218 Definition: The series of molecular signals generated as a consequence of the peptide neurotransmitter galanin binding to a cell surface receptor. References: PMID:25691535 Sources: GOC:lb Also known as: galanin-activated signalling pathway, galanin signaling pathway, galanin signalling pathway